{
  "gene_name": "Ubiquitin-conjugating enzyme E2 C",
  "gene": "UniProtKB:O00762",
  "gene_symbol": "UBE2C",
  "term_label": "protein polyubiquitination",
  "term_id": "GO:0000209"
}